stress-activated protein kinase signaling cascade [GO:0031098] (biological process) Also known as: SAPK signaling pathway, SAPK signalling pathway, stress-activated protein kinase signaling pathway, stress-activated protein kinase signalling pathway, JNK signaling pathway, JNK signalling pathway Relationships: is a type of cellular response to stress [GO:0033554]; is a type of intracellular signal transduction [GO:0035556] Subtypes: GO:0051403 Regulation: regulated by regulation of stress-activated protein kinase signaling cascade [GO:0070302]; negatively regulated by negative regulation of stress-activated protein kinase signaling cascade [GO:0070303]; positively regulated by positive regulation of stress-activated protein kinase signaling cascade [GO:0070304] Definition: The series of molecular signals in which a stress-activated protein kinase (SAPK) cascade relays a signal. Sources: GOC:mah